{
  "term_label": "G1/S transition of mitotic cell cycle",
  "term_id": "GO:0000082",
  "gene": "UniProtKB:Q86Y37",
  "gene_name": "CDK2-associated and cullin domain-containing protein 1",
  "gene_symbol": "CACUL1"
}